inositol phosphorylceramide synthase activity [GO:0102770] (molecular function) Relationships: is a type of phosphotransferase activity, alcohol group as acceptor [GO:0016773] Sources: MetaCyc:RXN-7795 Definition: Catalysis of the reaction: an L-1-phosphatidyl-inositol + a dihydroceramide = an inositol phosphodihydroceramide + a 1,2-diacyl-sn-glycerol.